positive regulation of AIM2 inflammasome complex assembly [GO:0140973] (biological process) References: PMID:33467177 Definition: Any process that activates or increases the frequency, rate or extent of AIM2 inflammasome complex assembly. Relationships: is_a positive regulation of protein-containing complex assembly [GO:0031334]; is a type of GO:0140971; is part of positive regulation of inflammasome-mediated signaling pathway [GO:0141087]; RO_0002213 AIM2 inflammasome complex assembly [GO:0140970]